{
  "gene_symbol": "MRPL16",
  "gene": "UniProtKB:Q9NX20",
  "gene_name": "Large ribosomal subunit protein uL16m",
  "term_id": "GO:0003735",
  "term_label": "structural constituent of ribosome"
}